{
  "term_label": "ryanodine-sensitive calcium-release channel activity",
  "gene": "UniProtKB:Q92736",
  "gene_name": "Ryanodine receptor 2",
  "gene_symbol": "RYR2",
  "term_id": "GO:0005219"
}